bundle sheath cell fate specification [GO:0090610] (BP) Relationships: is a type of cell fate specification [GO:0001708] Definition: The process in which a cell becomes capable of differentiating autonomously into a bundle sheath cell in an environment that is neutral with respect to the developmental pathway; upon specification, the cell fate can be reversed. References: PMID:24517883 Sources: GOC:tb